protein localization to chromatin [GO:0071168] (biological process) Definition: Any process in which a protein is transported to, or maintained at, a part of a chromosome that is organized into chromatin. Sources: GOC:mah Also known as: protein localisation to chromatin Relationships: is a type of protein localization to chromosome [GO:0034502] Subtypes: protein localization to CENP-A containing chromatin [GO:0061644], protein localization to heterochromatin [GO:0097355], protein localization to euchromatin [GO:1905632] Regulation: negatively regulated by GO:0120186; positively regulated by positive regulation of protein localization to chromatin [GO:0120187]; regulated by regulation of protein localization to chromatin [GO:1905634]